positive regulation of cell communication [GO:0010647] (biological process) Subtypes: positive regulation of signal transduction [GO:0009967], positive regulation of cell communication by electrical coupling [GO:0010650], positive regulation of cell communication by chemical coupling [GO:0010652], positive regulation of hormone secretion [GO:0046887], positive regulation of synaptic transmission [GO:0050806], positive regulation of transmission of nerve impulse [GO:0051971], positive regulation of Wnt protein secretion [GO:0061357], GO:0061941, positive regulation of BMP secretion [GO:1900144], positive regulation of retrograde trans-synaptic signaling by neuropeptide [GO:1905434] Definition: Any process that increases the frequency, rate or extent of cell communication. Cell communication is the process that mediates interactions between a cell and its surroundings. Encompasses interactions such as signaling or attachment between one cell and another cell, between a cell and an extracellular matrix, or between a cell and any other aspect of its environment. Sources: GOC:dph, GOC:tb Relationships: is_a regulation of cell communication [GO:0010646]; is a type of positive regulation of cellular process [GO:0048522]; positively regulates cell communication [GO:0007154]